face morphogenesis [GO:0060325] (biological process) Definition: The process in which the anatomical structures of the face are generated and organized. The face is the ventral division of the head. Relationships: is a type of anatomical structure morphogenesis [GO:0009653]; is part of head morphogenesis [GO:0060323]; is part of face development [GO:0060324] Sources: GOC:dph